regulation of calcium ion-dependent exocytosis of neurotransmitter [GO:1903233] (biological process) References: PMID:16782817 Sources: GOC:TermGenie, GO_REF:0000058 Definition: Any process that modulates the frequency, rate or extent of calcium ion-dependent exocytosis of neurotransmitter. Note: An example of this is Rab3gap1 in mouse (Q80UJ7) in PMID:16782817 (IMP) Subtypes: regulation of presynaptic dense core granule exocytosis [GO:0099161], negative regulation of calcium ion-dependent exocytosis of neurotransmitter [GO:1903234], positive regulation of calcium ion-dependent exocytosis of neurotransmitter [GO:1903235] Relationships: is a type of regulation of calcium ion-dependent exocytosis [GO:0017158]; is a type of GO:2000300; regulates calcium ion-regulated exocytosis of neurotransmitter [GO:0048791]